{
  "term_id": "GO:0001227",
  "gene_symbol": "ZBTB10",
  "gene": "UniProtKB:Q96DT7",
  "term_label": "DNA-binding transcription repressor activity, RNA polymerase II-specific",
  "gene_name": "Zinc finger and BTB domain-containing protein 10"
}